melanocortin receptor activity [GO:0004977] (molecular function) Definition: Combining with melanocortin to initiate a change in cell activity. Sources: GOC:ai Relationships: is a type of G protein-coupled peptide receptor activity [GO:0008528] Subtypes: corticotropin receptor activity [GO:0004978], beta-endorphin receptor activity [GO:0004979], melanocyte-stimulating hormone receptor activity [GO:0004980]